{
  "gene_name": "Alcohol dehydrogenase class-3",
  "gene": "UniProtKB:P11766",
  "gene_symbol": "ADH5",
  "term_id": "GO:0008270",
  "term_label": "zinc ion binding"
}